protein homodimerization activity [GO:0042803] (molecular function) Also known as: dimerization activity Definition: Binding to an identical protein to form a homodimer. Sources: GOC:jl Relationships: is a type of identical protein binding [GO:0042802]; is a type of protein dimerization activity [GO:0046983]